dosage compensation complex [GO:0046536] (cellular component) Definition: A protein or protein-RNA complex that localizes to one or more of the sex chromosome(s), where it acts to normalize transcription between different sexes. Relationships: is a type of nuclear protein-containing complex [GO:0140513]; is part of GO:0000785; is part of GO:0000803 Subtypes: X chromosome located dosage compensation complex, transcription activating [GO:0016456] Sources: GOC:kmv, GOC:mah